{
  "gene": "UniProtKB:P55899",
  "term_label": "beta-2-microglobulin binding",
  "gene_symbol": "FCGRT",
  "term_id": "GO:0030881",
  "gene_name": "IgG receptor FcRn large subunit p51"
}